{
  "term_label": "zinc chaperone activity",
  "gene_symbol": "ZNG1C",
  "gene": "UniProtKB:Q5JTY5",
  "gene_name": "Zinc-regulated GTPase metalloprotein activator 1C",
  "term_id": "GO:0140827"
}